membrane addition at site of cytokinesis [GO:0007107] (biological process) Sources: GOC:clt Subtypes: membrane addition at site of mitotic cytokinesis [GO:0061796] Definition: Any process involved in the net addition of membrane at the site of cytokinesis; includes vesicle recruitment and fusion, local lipid synthesis and insertion. Also known as: cytokinesis, membrane recruitment/generation Relationships: is a type of cytokinetic process [GO:0032506]; is a type of membrane organization [GO:0061024]